{
  "gene_symbol": "PLXNA4",
  "term_id": "GO:0030334",
  "gene": "UniProtKB:Q9HCM2",
  "term_label": "regulation of cell migration",
  "gene_name": "Plexin-A4"
}